{
  "term_label": "cytosol",
  "term_id": "GO:0005829",
  "gene_name": "Peptidyl-prolyl cis-trans isomerase FKBP8",
  "gene_symbol": "FKBP8",
  "gene": "UniProtKB:Q14318"
}